{
  "term_id": "GO:0005886",
  "term_label": "plasma membrane",
  "gene_symbol": "LPAR3",
  "gene_name": "Lysophosphatidic acid receptor 3",
  "gene": "UniProtKB:Q9UBY5"
}